amidinoaspartase activity [GO:0047660] (MF) Definition: Catalysis of the reaction: N-amidino-L-aspartate + H2O = L-aspartate + urea. Also known as: N-amidino-L-aspartate amidinohydrolase activity, amidinoaspartic amidinohydrolase activity Sources: EC:3.5.3.14, RHEA:14849 Relationships: is a type of GO:0016813